{
  "term_id": "GO:0030335",
  "term_label": "positive regulation of cell migration",
  "gene": "UniProtKB:Q9GZP0",
  "gene_name": "Platelet-derived growth factor D",
  "gene_symbol": "PDGFD"
}